{
  "gene_symbol": "DNAAF5",
  "gene_name": "Dynein axonemal assembly factor 5",
  "gene": "UniProtKB:Q86Y56",
  "term_id": "GO:0036158",
  "term_label": "outer dynein arm assembly"
}